{
  "gene_name": "Pericentrin",
  "term_label": "Unknown molecular function",
  "gene_symbol": "PCNT",
  "term_id": "UNKNOWN:0001",
  "gene": "UniProtKB:O95613"
}